{
  "term_label": "cilium assembly",
  "term_id": "GO:0060271",
  "gene_name": "Cilium assembly protein DZIP1L",
  "gene": "UniProtKB:Q8IYY4",
  "gene_symbol": "DZIP1L"
}